{
  "gene": "UniProtKB:Q5TAH2",
  "term_label": "potassium:proton antiporter activity",
  "term_id": "GO:0015386",
  "gene_symbol": "SLC9C2",
  "gene_name": "Sodium_hydrogen exchanger 11"
}